nuclear viral factory [GO:0039715] (cellular component) Definition: A viral factory located in the nucleus of a host cell. Subtypes: GO:0039720, GO:0039721, replication compartment [GO:0046809] Relationships: is a type of viral factory [GO:0039713]; is part of host cell nucleus [GO:0042025] Sources: VZ:1951